{
  "term_label": "RNA polymerase II cis-regulatory region sequence-specific DNA binding",
  "gene_name": "Nuclear receptor subfamily 1 group D member 2",
  "gene_symbol": "NR1D2",
  "term_id": "GO:0000978",
  "gene": "UniProtKB:Q14995"
}